{
  "term_id": "GO:0005634",
  "term_label": "nucleus",
  "gene_symbol": "ELF3",
  "gene_name": "ETS-related transcription factor Elf-3",
  "gene": "UniProtKB:P78545"
}